L-iduronidase activity [GO:0003940] (molecular function) Also known as: alpha-L-iduronidase activity, glycosaminoglycan alpha-L-iduronohydrolase activity Definition: Catalysis of the hydrolysis of alpha-L-iduronosidic linkages in dermatan sulfate. Can also hydrolyze alpha-L-iduronosidic linkages in heparan sulfate. Relationships: is_a hydrolase activity, hydrolyzing O-glycosyl compounds [GO:0004553] References: PMID:35011691 Sources: EC:3.2.1.76